{
  "gene_name": "Frizzled-4",
  "gene_symbol": "FZD4",
  "gene": "UniProtKB:Q9ULV1",
  "term_id": "GO:0035567",
  "term_label": "non-canonical Wnt signaling pathway"
}